{
  "term_id": "GO:0006741",
  "gene_symbol": "NADK",
  "term_label": "NADP+ biosynthetic process",
  "gene": "UniProtKB:O95544",
  "gene_name": "NAD kinase"
}